GET complex [GO:0043529] (cellular component) Definition: An endoplasmic reticulum protein-containing complex that is conserved in eukaryotics and that mediates the insertion of tail-anchored proteins into the ER membrane. In yeast, includes Get1p, Get2p and Get3p proteins. References: PMID:16269340, PMID:18724936, PMID:32910895 Sources: GOC:krc, GOC:vw Relationships: is a type of GO:0140534